{
  "gene_name": "HLA class II histocompatibility antigen, DO alpha chain",
  "gene": "UniProtKB:P06340",
  "term_id": "GO:0031902",
  "term_label": "late endosome membrane",
  "gene_symbol": "HLA-DOA"
}